{
  "gene_name": "Zinc finger protein 296",
  "gene_symbol": "ZNF296",
  "gene": "UniProtKB:Q8WUU4",
  "term_id": "GO:0006357",
  "term_label": "regulation of transcription by RNA polymerase II"
}